{
  "gene_symbol": "CHEK2",
  "gene_name": "Serine_threonine-protein kinase Chk2",
  "gene": "UniProtKB:O96017",
  "term_id": "GO:0004674",
  "term_label": "protein serine/threonine kinase activity"
}